{
  "gene_name": "Phosphatidylinositol-binding clathrin assembly protein",
  "gene_symbol": "PICALM",
  "term_label": "clathrin-coated pit",
  "gene": "UniProtKB:Q13492",
  "term_id": "GO:0005905"
}